{
  "term_id": "GO:0007015",
  "term_label": "actin filament organization",
  "gene_name": "Unconventional myosin-Ia",
  "gene_symbol": "MYO1A",
  "gene": "UniProtKB:Q9UBC5"
}